{
  "term_id": "GO:0098978",
  "gene_name": "Caskin-1",
  "term_label": "glutamatergic synapse",
  "gene": "UniProtKB:Q8WXD9",
  "gene_symbol": "CASKIN1"
}